mitochondrial isopropylmalate transmembrane transport [GO:1990556] (BP) References: PMID:10428783 Relationships: is a type of 2-isopropylmalate(2-) transmembrane transport [GO:1902357] Definition: The process in which 2-isopropylmalate(2-) is transported across a mitochondrial membrane, into or out of the mitochondrion.